{
  "term_label": "peptidyl-prolyl cis-trans isomerase activity",
  "term_id": "GO:0003755",
  "gene": "UniProtKB:Q9UNP9",
  "gene_symbol": "PPIE",
  "gene_name": "Peptidyl-prolyl cis-trans isomerase E"
}